{
  "gene_name": "Mannosyl-oligosaccharide 1,2-alpha-mannosidase IA",
  "gene": "UniProtKB:P33908",
  "gene_symbol": "MAN1A1",
  "term_label": "ERAD pathway",
  "term_id": "GO:0036503"
}